{
  "gene": "UniProtKB:Q8N693",
  "gene_name": "Homeobox protein ESX1",
  "term_id": "GO:0005634",
  "gene_symbol": "ESX1",
  "term_label": "nucleus"
}